{
  "term_id": "GO:0006955",
  "gene": "UniProtKB:P04433",
  "term_label": "immune response",
  "gene_symbol": "IGKV3-11",
  "gene_name": "Immunoglobulin kappa variable 3-11"
}